cellular response to boron-containing substance deprivation [GO:0080169] (biological process) Relationships: is a type of cellular response to starvation [GO:0009267]; is a type of cellular response to chemical stress [GO:0062197]; is a type of cellular response to boron-containing substance levels [GO:0080029] References: PMID:20059736 Definition: Any process that results in a change in state or activity of a cell (in terms of movement, secretion, enzyme production, gene expression, etc.) as a result of deprivation of boron obtained from boron-containing substances. Also known as: cellular response to boron deprivation, cellular response to boron starvation